convergent extension involved in metanephric nephron morphogenesis [GO:0072279] (biological process) Sources: GOC:mtg_kidney_jan10 Relationships: is a type of convergent extension involved in nephron morphogenesis [GO:0072045]; is part of GO:0072273 Definition: The morphogenetic process in which the renal epithelium narrows along one axis and lengthens in a perpendicular axis that contributes to the shaping of a nephron in the metanephros.